{
  "term_label": "proteasome core complex, alpha-subunit complex",
  "gene": "UniProtKB:O14818",
  "term_id": "GO:0019773",
  "gene_name": "Proteasome subunit alpha type-7",
  "gene_symbol": "PSMA7"
}